{
  "term_id": "GO:0036126",
  "gene_symbol": "SAXO1",
  "gene": "UniProtKB:Q8IYX7",
  "term_label": "sperm flagellum",
  "gene_name": "Stabilizer of axonemal microtubules 1"
}